{
  "term_label": "Unknown biological process",
  "gene": "UniProtKB:A0A590UK83",
  "term_id": "UNKNOWN:0002",
  "gene_name": "Small integral membrane protein 45",
  "gene_symbol": "SMIM45"
}